{
  "gene": "UniProtKB:Q3LI63",
  "gene_name": "Keratin-associated protein 20-1",
  "term_id": "UNKNOWN:0001",
  "term_label": "Unknown molecular function",
  "gene_symbol": "KRTAP20-1"
}